optic vesicle morphogenesis [GO:0003404] (biological process) Relationships: is a type of GO:0048598; is a type of tissue morphogenesis [GO:0048729]; is part of embryonic camera-type eye morphogenesis [GO:0048596] Definition: The developmental process pertaining to the formation and shaping of the optic vesicle. This process begins with the specific processes that contribute to the appearance of the vesicle and ends when the vesicle has evaginated. The optic vesicle is the evagination of neurectoderm that precedes formation of the optic cup. Sources: GOC:ascb_2009, GOC:dph, GOC:tb